{
  "gene_name": "Transforming protein RhoA",
  "gene_symbol": "RHOA",
  "term_id": "GO:0016477",
  "gene": "UniProtKB:P61586",
  "term_label": "cell migration"
}